prostaglandin binding [GO:1904593] (molecular function) Definition: Binding to prostaglandin. References: PMID:21445266 Sources: GOC:TermGenie, GO_REF:0000067 Relationships: is a type of fatty acid derivative binding [GO:1901567]